{
  "gene_symbol": "CLIC5",
  "term_label": "Unknown biological process",
  "gene_name": "Chloride intracellular channel protein 5",
  "term_id": "UNKNOWN:0002",
  "gene": "UniProtKB:Q9NZA1"
}